{
  "term_id": "GO:0006357",
  "gene": "UniProtKB:Q8TAW3",
  "gene_name": "Zinc finger protein 671",
  "term_label": "regulation of transcription by RNA polymerase II",
  "gene_symbol": "ZNF671"
}